{
  "gene_symbol": "FANCD2OS",
  "gene": "UniProtKB:Q96PS1",
  "term_id": "UNKNOWN:0001",
  "term_label": "Unknown molecular function",
  "gene_name": "FANCD2 opposite strand protein"
}